{
  "gene": "UniProtKB:Q5VTE6",
  "term_id": "GO:0003730",
  "gene_name": "Protein angel homolog 2",
  "term_label": "mRNA 3'-UTR binding",
  "gene_symbol": "ANGEL2"
}